prostate gland morphogenetic growth [GO:0060737] (biological process) Sources: GOC:dph Definition: The differential increase in size or mass of the prostate gland that contributes to the gland attaining its form. Subtypes: primary prostatic bud elongation [GO:0060516], prostate epithelial cord elongation [GO:0060523] Relationships: is a type of developmental growth involved in morphogenesis [GO:0060560]; is_a GO:0060736; is part of prostate gland morphogenesis [GO:0060512] Also known as: prostate gland growth involved in morphogenesis